{
  "gene": "UniProtKB:P59046",
  "term_id": "GO:0050727",
  "term_label": "regulation of inflammatory response",
  "gene_name": "NACHT, LRR and PYD domains-containing protein 12",
  "gene_symbol": "NLRP12"
}